establishment of meiotic spindle orientation [GO:0051296] (biological process) Sources: GOC:ai Also known as: establishment of spindle orientation involved in meiotic cell cycle, meiotic spindle orientation, orienting of meiotic spindle, establishment of spindle orientation during meiosis Relationships: is a type of establishment of spindle orientation [GO:0051294]; is_a establishment of meiotic spindle localization [GO:0051295] Definition: Any process that set the alignment of meiotic spindle relative to other cellular structures.